{
  "gene": "UniProtKB:W6CW81",
  "gene_name": "Pyrin domain-containing protein 5",
  "gene_symbol": "PYDC5",
  "term_id": "UNKNOWN:0003",
  "term_label": "Unknown cellular component"
}